{
  "term_id": "UNKNOWN:0001",
  "gene_name": "CBY1-interacting BAR domain-containing protein 2",
  "term_label": "Unknown molecular function",
  "gene": "UniProtKB:Q6ZTR7",
  "gene_symbol": "CIBAR2"
}